{
  "term_id": "UNKNOWN:0002",
  "gene": "UniProtKB:Q96M91",
  "term_label": "Unknown biological process",
  "gene_name": "Cilia- and flagella-associated protein 53",
  "gene_symbol": "CFAP53"
}